{
  "term_label": "retina development in camera-type eye",
  "term_id": "GO:0060041",
  "gene_symbol": "PDE6B",
  "gene_name": "Rod cGMP-specific 3',5'-cyclic phosphodiesterase subunit beta",
  "gene": "UniProtKB:P35913"
}